{
  "gene": "UniProtKB:P62079",
  "term_id": "UNKNOWN:0002",
  "gene_symbol": "TSPAN5",
  "gene_name": "Tetraspanin-5",
  "term_label": "Unknown biological process"
}